secretion by cell [GO:0032940] (biological process) Regulation: regulated by regulation of secretion by cell [GO:1903530]; negatively regulated by GO:1903531; positively regulated by positive regulation of secretion by cell [GO:1903532] Subtypes: exocytosis [GO:0006887], protein secretion [GO:0009306], GO:0010585, glutamate secretion [GO:0014047], GO:0023061, secretion by the type IV secretion system [GO:0044097], GO:0050432, secretion by lung epithelial cell involved in lung growth [GO:0061033], aspartate secretion [GO:0061528], primary amine secretion [GO:0061531], glycine secretion [GO:0061536], octopamine secretion [GO:0061539], extracellular matrix constituent secretion [GO:0070278] Also known as: cellular secretion Definition: The controlled release of a substance by a cell. Relationships: is a type of secretion [GO:0046903]; is_a export from cell [GO:0140352] Sources: GOC:mah